spermine transport [GO:0000296] (biological process) Subtypes: spermine transmembrane transport [GO:1903710] Definition: The directed movement of spermine, N,N-bis(3-aminopropyl)-1,4-diaminobutane, a polyamine formed by the transfer of a propylamine group from decarboxylated S-adenosylmethionine to spermidine, into, out of or within a cell, or between cells, by means of some agent such as a transporter or pore. Sources: GOC:krc, ISBN:0198506732 Relationships: is a type of polyamine transport [GO:0015846]